{
  "gene": "UniProtKB:A0A1B0GVR7",
  "term_id": "UNKNOWN:0002",
  "gene_name": "Protein FAM240C",
  "gene_symbol": "FAM240C",
  "term_label": "Unknown biological process"
}